diadenosine hexaphosphate catabolic process [GO:1901909] (BP) Relationships: is a type of diadenosine polyphosphate catabolic process [GO:0015961] Definition: The chemical reactions and pathways resulting in the breakdown of diadenosine hexaphosphate. References: PMID:10090752 Sources: GOC:TermGenie Also known as: diadenosine hexaphosphate catabolism, diadenosyl hexaphosphate breakdown, diadenosyl hexaphosphate catabolic process, diadenosyl hexaphosphate catabolism, diadenosyl hexaphosphate degradation